{
  "gene_name": "Large ribosomal subunit protein bL9m",
  "term_id": "UNKNOWN:0002",
  "gene": "UniProtKB:Q9BYD2",
  "gene_symbol": "MRPL9",
  "term_label": "Unknown biological process"
}